{
  "gene_symbol": "PWWP2A",
  "gene_name": "PWWP domain-containing protein 2A",
  "gene": "UniProtKB:Q96N64",
  "term_label": "Unknown biological process",
  "term_id": "UNKNOWN:0002"
}